{
  "term_label": "cell migration",
  "gene_name": "Serine_threonine-protein kinase PAK 3",
  "gene_symbol": "PAK3",
  "gene": "UniProtKB:O75914",
  "term_id": "GO:0016477"
}